{
  "gene": "UniProtKB:Q8NDF8",
  "term_label": "nucleolus",
  "term_id": "GO:0005730",
  "gene_name": "Terminal nucleotidyltransferase 4B",
  "gene_symbol": "TENT4B"
}